{
  "gene": "UniProtKB:Q9NRC8",
  "gene_symbol": "SIRT7",
  "gene_name": "NAD-dependent protein deacetylase sirtuin-7",
  "term_id": "GO:0140861",
  "term_label": "DNA repair-dependent chromatin remodeling"
}